{
  "term_id": "GO:0016020",
  "gene_name": "Chloride intracellular channel protein 1",
  "gene_symbol": "CLIC1",
  "term_label": "membrane",
  "gene": "UniProtKB:O00299"
}